cellular response to UV-C [GO:0071494] (BP) Sources: GOC:mah Definition: Any process that results in a change in state or activity of a cell (in terms of movement, secretion, enzyme production, gene expression, etc.) as a result of a UV-C radiation stimulus. UV-C radiation (UV-C light) spans the wavelengths 100 to 280 nm. Relationships: is a type of response to UV-C [GO:0010225]; is a type of cellular response to UV [GO:0034644] Also known as: cellular response to UV-C light stimulus, cellular response to UV-C radiation stimulus, cellular response to UVC light stimulus, cellular response to UVC radiation stimulus, cellular response to germicidal ultraviolet light stimulus, cellular response to germicidal ultraviolet radiation stimulus, cellular response to shortwave ultraviolet light stimulus, cellular response to shortwave ultraviolet radiation stimulus